negative regulation of zoospore encystment on host [GO:0075221] (BP) Sources: GOC:pamgo_curators Relationships: is a type of negative regulation of spore encystment on host [GO:0075217]; is a type of GO:0075219; RO_0002212 zoospore encystment on host [GO:0075218] Definition: Any process that stops, prevents, or reduces the frequency, rate or extent of zoospore encystment on host. The host is defined as the larger of the organisms involved in a symbiotic interaction.